{
  "term_label": "extracellular space",
  "term_id": "GO:0005615",
  "gene": "UniProtKB:P48023",
  "gene_symbol": "FASLG",
  "gene_name": "Tumor necrosis factor ligand superfamily member 6"
}